{
  "term_id": "GO:0043679",
  "gene": "UniProtKB:Q14003",
  "gene_symbol": "KCNC3",
  "term_label": "axon terminus",
  "gene_name": "Potassium voltage-gated channel subfamily C member 3"
}